{
  "gene_symbol": "CD48",
  "gene": "UniProtKB:P09326",
  "term_label": "Unknown cellular component",
  "term_id": "UNKNOWN:0003",
  "gene_name": "CD48 antigen"
}